{
  "term_label": "commissural neuron axon guidance",
  "gene": "UniProtKB:Q99835",
  "term_id": "GO:0071679",
  "gene_symbol": "SMO",
  "gene_name": "Protein smoothened"
}